phosphoarginine biosynthetic process [GO:0046312] (biological process) Relationships: is a type of phosphagen biosynthetic process [GO:0042396]; is a type of GO:0170034; is_a non-proteinogenic amino acid biosynthetic process [GO:0170043] Definition: The chemical reactions and pathways resulting in the formation of phosphoarginine, a phosphorylated derivative of the amino acid arginine. Sources: GOC:ai Also known as: phosphoarginine anabolism, phosphoarginine biosynthesis, phosphoarginine formation, phosphoarginine synthesis